{
  "gene_name": "E3 ubiquitin-protein ligase UBR1",
  "gene_symbol": "UBR1",
  "term_id": "GO:0000151",
  "term_label": "ubiquitin ligase complex",
  "gene": "UniProtKB:Q8IWV7"
}